{
  "term_label": "regulation of glycolytic process",
  "term_id": "GO:0006110",
  "gene": "UniProtKB:P54619",
  "gene_name": "5'-AMP-activated protein kinase subunit gamma-1",
  "gene_symbol": "PRKAG1"
}